{
  "gene": "UniProtKB:P48436",
  "term_id": "GO:0000978",
  "gene_symbol": "SOX9",
  "gene_name": "Transcription factor SOX-9",
  "term_label": "RNA polymerase II cis-regulatory region sequence-specific DNA binding"
}